maternal determination of anterior/posterior axis, embryo [GO:0008358] (biological process) Sources: ISBN:0879694238, http://fly.ebi.ac.uk/allied-data/lk/interactive-fly/aimain/1aahome.htm Relationships: is a type of anterior/posterior axis specification, embryo [GO:0008595] Definition: The specification of the anterior/posterior axis of the embryo by gradients of maternally-transcribed gene products; exemplified in insects by the morphogens, bicoid and nanos.